{
  "term_label": "antigen binding",
  "gene_symbol": "IGLL5",
  "gene_name": "Immunoglobulin lambda-like polypeptide 5",
  "term_id": "GO:0003823",
  "gene": "UniProtKB:B9A064"
}